histone H3K9me/H3K9me2 demethylase activity [GO:0140683] (molecular function) Note: Comment: Note that the residue position corresponds to the canonical human H3 histone (UniProtKB:P84243); this residue is conserved across all eukaryotes. Residue 1 is the first residue following removal of the initiating Methionine (Met). Note that each histone is encoded by multiple genes, and sequences may vary across different genes within an organism. Also known as: histone H3K9me demethylase activity, histone H3K9me2 demethylase activity, histone H3-di/monomethyl-lysine-9 demethylase activity Relationships: is a type of GO:0016706; is a type of GO:0032454 References: PMID:16603238 Definition: Catalysis of the removal of a methyl group from a di or a monomethyl-lysine residue at position 9 of the histone H3 protein. This is a dioxygenase reaction that is dependent on Fe(II) and 2-oxoglutarate.